{
  "term_id": "UNKNOWN:0001",
  "gene_symbol": "RAB11FIP4",
  "term_label": "Unknown molecular function",
  "gene": "UniProtKB:Q86YS3",
  "gene_name": "Rab11 family-interacting protein 4"
}